pupariation [GO:0035073] (biological process) References: PMID:9409683 Sources: GOC:bf, ISBN:0879694238 Relationships: is a type of GO:0032501; is part of prepupal development [GO:0035210] Also known as: puparium biosynthesis, puparium formation Definition: The onset of prepupal development when the larval stops crawling, everts its spiracles and the larval cuticle becomes the puparium or pupal case that surrounds the organism for the duration of metamorphosis. Regulation: regulated by GO:0106023; negatively regulated by negative regulation of pupariation [GO:0106024]; positively regulated by positive regulation of pupariation [GO:0106025]